{
  "gene_symbol": "SOD1",
  "gene_name": "Superoxide dismutase [Cu-Zn]",
  "term_label": "mitochondrion",
  "term_id": "GO:0005739",
  "gene": "UniProtKB:P00441"
}